{
  "gene": "UniProtKB:Q8N2C9",
  "gene_symbol": "UMODL1-AS1",
  "term_id": "UNKNOWN:0002",
  "term_label": "Unknown biological process",
  "gene_name": "Uncharacterized protein UMODL1-AS1"
}